{
  "gene_symbol": "TCEAL6",
  "gene": "UniProtKB:Q6IPX3",
  "gene_name": "Transcription elongation factor A protein-like 6",
  "term_label": "Unknown cellular component",
  "term_id": "UNKNOWN:0003"
}